negative regulation of centrosome cycle [GO:0046606] (biological process) Definition: Any process that stops, prevents, or reduces the frequency, rate or extent of the centrosome cycle. Subtypes: negative regulation of centrosome duplication [GO:0010826] Sources: GOC:ai Relationships: is a type of negative regulation of cell cycle process [GO:0010948]; is a type of GO:0046605; is a type of negative regulation of cytoskeleton organization [GO:0051494]; negatively regulates GO:0007098 Also known as: down regulation of centrosome cycle, down-regulation of centrosome cycle, downregulation of centrosome cycle, inhibition of centrosome cycle